{
  "gene_name": "StAR-related lipid transfer protein 5",
  "term_id": "GO:0015485",
  "term_label": "cholesterol binding",
  "gene_symbol": "STARD5",
  "gene": "UniProtKB:Q9NSY2"
}